{
  "gene": "UniProtKB:Q8NGM9",
  "term_id": "GO:0007186",
  "term_label": "G protein-coupled receptor signaling pathway",
  "gene_name": "Olfactory receptor 8D4",
  "gene_symbol": "OR8D4"
}